negative regulation of plasma membrane raft polarization [GO:1903907] (biological process) Also known as: down regulation of plasma membrane raft polarization, down-regulation of plasma membrane raft polarization, downregulation of plasma membrane raft polarization, inhibition of plasma membrane raft polarization References: PMID:23575248 Sources: GOC:TermGenie, GOC:als, GO_REF:0000058 Relationships: is a type of negative regulation of cellular component organization [GO:0051129]; is a type of regulation of plasma membrane raft polarization [GO:1903906]; negatively regulates plasma membrane raft polarization [GO:0044858] Definition: Any process that stops, prevents or reduces the frequency, rate or extent of plasma membrane raft polarization.